{
  "term_label": "deoxyribonuclease I activity",
  "gene_name": "Deoxyribonuclease-1",
  "term_id": "GO:0004530",
  "gene": "UniProtKB:P24855",
  "gene_symbol": "DNASE1"
}